{
  "gene_name": "Acyl-CoA-binding domain-containing protein 5",
  "term_id": "GO:0005777",
  "gene_symbol": "ACBD5",
  "gene": "UniProtKB:Q5T8D3",
  "term_label": "peroxisome"
}